{
  "gene_name": "Tyrosine-protein kinase Yes",
  "term_id": "GO:0005886",
  "gene_symbol": "YES1",
  "term_label": "plasma membrane",
  "gene": "UniProtKB:P07947"
}